{
  "gene": "UniProtKB:Q6ZTQ3",
  "term_id": "UNKNOWN:0001",
  "term_label": "Unknown molecular function",
  "gene_symbol": "RASSF6",
  "gene_name": "Ras association domain-containing protein 6"
}